{
  "gene_symbol": "CELF3",
  "term_id": "GO:0000381",
  "gene": "UniProtKB:Q5SZQ8",
  "term_label": "regulation of alternative mRNA splicing, via spliceosome",
  "gene_name": "CUGBP Elav-like family member 3"
}